{
  "gene": "UniProtKB:O75690",
  "gene_name": "Keratin-associated protein 5-8",
  "gene_symbol": "KRTAP5-8",
  "term_label": "Unknown cellular component",
  "term_id": "UNKNOWN:0003"
}